{
  "term_id": "GO:0005615",
  "term_label": "extracellular space",
  "gene": "UniProtKB:Q02985",
  "gene_name": "Complement factor H-related protein 3",
  "gene_symbol": "CFHR3"
}